{
  "gene": "UniProtKB:Q96D59",
  "gene_name": "E3 ubiquitin-protein ligase RNF183",
  "term_label": "positive regulation of endoplasmic reticulum stress-induced intrinsic apoptotic signaling pathway",
  "gene_symbol": "RNF183",
  "term_id": "GO:1902237"
}